{
  "term_label": "dynein complex",
  "gene_name": "Dynein axonemal heavy chain 10",
  "gene_symbol": "DNAH10",
  "term_id": "GO:0030286",
  "gene": "UniProtKB:Q8IVF4"
}